{
  "term_id": "GO:0043015",
  "gene": "UniProtKB:Q96SN8",
  "gene_symbol": "CDK5RAP2",
  "gene_name": "CDK5 regulatory subunit-associated protein 2",
  "term_label": "gamma-tubulin binding"
}